skin epidermis development [GO:0098773] (biological process) Definition: The process whose specific outcome is the progression of the skin epidermis over time, from its formation to the mature structure. Sources: GOC:dos Relationships: is a type of epidermis development [GO:0008544]; is_a GO:0060429; BFO_0000050 skin development [GO:0043588] Subtypes: limb epidermis development [GO:0060887], GO:0061436